plasmacytoid dendritic cell antigen processing and presentation [GO:0002470] (biological process) Definition: The process in which a plasmacytoid dendritic cell expresses antigen (peptide or lipid) on its cell surface in association with an MHC protein complex. References: PMID:15771591 Sources: GOC:add, ISBN:0781735149 Relationships: is a type of GO:0002468 Regulation: regulated by GO:0002610; negatively regulated by negative regulation of plasmacytoid dendritic cell antigen processing and presentation [GO:0002611]; positively regulated by GO:0002612